{
  "gene_symbol": "HOXA1",
  "term_label": "DNA-binding transcription factor activity, RNA polymerase II-specific",
  "term_id": "GO:0000981",
  "gene": "UniProtKB:P49639",
  "gene_name": "Homeobox protein Hox-A1"
}